{
  "term_id": "GO:0046323",
  "gene": "UniProtKB:Q9NRM0",
  "term_label": "D-glucose import",
  "gene_name": "Solute carrier family 2, facilitated glucose transporter member 9",
  "gene_symbol": "SLC2A9"
}